{
  "term_label": "erythrocyte differentiation",
  "gene": "UniProtKB:Q8IX07",
  "gene_symbol": "ZFPM1",
  "term_id": "GO:0030218",
  "gene_name": "Zinc finger protein ZFPM1"
}